F420-0 metabolic process [GO:0052645] (biological process) Also known as: F(420)-0 metabolic process, F420-0 metabolism, coenzyme F420-0 metabolic process, coenzyme F420-0 metabolism Definition: The chemical reactions and pathways involving F420-0 (5-O-{[(1S)-1-carboxyethoxy](hydroxy)phosphoryl}-1-deoxy-1-(8-hydroxy-2,4-dioxo-2H-pyrimido[4,5-b]quinolin-10(4H)-yl)-D-ribitol), the fragment of coenzyme F420 remaining after formal hydrolytic removal of all of the glutamate residues. Sources: GOC:curators Relationships: is a type of monocarboxylic acid metabolic process [GO:0032787]; is a type of GO:0052646